{
  "gene": "UniProtKB:P08582",
  "gene_symbol": "MELTF",
  "gene_name": "Melanotransferrin",
  "term_label": "early endosome",
  "term_id": "GO:0005769"
}